angiogenesis involved in wound healing [GO:0060055] (biological process) Subtypes: vascular wound healing [GO:0061042] Relationships: is a type of angiogenesis [GO:0001525]; is part of GO:0042060 References: PMID:15039218 Sources: GOC:dph Definition: Blood vessel formation when new vessels emerge from the proliferation of pre-existing blood vessels and contribute to the series of events that restore integrity to a damaged tissue, following an injury.